{
  "gene": "UniProtKB:P55085",
  "gene_symbol": "F2RL1",
  "gene_name": "Proteinase-activated receptor 2",
  "term_id": "GO:0007186",
  "term_label": "G protein-coupled receptor signaling pathway"
}